endocrine system development [GO:0035270] (biological process) Sources: GOC:bf, Wikipedia:Development_of_the_endocrine_system Relationships: is a type of GO:0048731 Definition: Progression of the endocrine system over time, from its formation to a mature structure. The endocrine system is a system of hormones and ductless glands, where the glands release hormones directly into the blood, lymph or other intercellular fluid, and the hormones circulate within the body to affect distant organs. The major glands that make up the human endocrine system are the hypothalamus, pituitary, thyroid, parathryoids, adrenals, pineal body, and the reproductive glands which include the ovaries and testes.